{
  "term_id": "GO:0030182",
  "gene_name": "Insulinoma-associated protein 2",
  "gene_symbol": "INSM2",
  "gene": "UniProtKB:Q96T92",
  "term_label": "neuron differentiation"
}